{
  "gene_symbol": "COL8A1",
  "term_id": "GO:0031012",
  "gene_name": "Collagen alpha-1(VIII) chain",
  "gene": "UniProtKB:P27658",
  "term_label": "extracellular matrix"
}